{
  "term_id": "GO:0005615",
  "term_label": "extracellular space",
  "gene": "UniProtKB:O00253",
  "gene_name": "Agouti-related protein",
  "gene_symbol": "AGRP"
}